{
  "term_id": "GO:0015297",
  "gene_symbol": "SLC35E3",
  "gene_name": "Solute carrier family 35 member E3",
  "gene": "UniProtKB:Q7Z769",
  "term_label": "antiporter activity"
}